{
  "term_id": "GO:0090443",
  "gene_name": "Striatin",
  "term_label": "FAR/SIN/STRIPAK complex",
  "gene_symbol": "STRN",
  "gene": "UniProtKB:O43815"
}